inflorescence phyllotactic patterning [GO:0090643] (biological process) Definition: The radial pattern formation process that results in the formation of flowers around a central axis in an inflorescence meristem. References: PMID:25352850 Relationships: is a type of phyllotactic patterning [GO:0060771]